detection of stimulus involved in sensory perception of pain [GO:0062149] (biological process) Definition: The series of events involved in the perception of pain in which a stimulus is received and converted into a molecular signal. References: PMID:19837031 Relationships: is_a GO:0050906; BFO_0000050 GO:0019233 Subtypes: detection of temperature stimulus involved in sensory perception of pain [GO:0050965], GO:0050966, GO:0050967, detection of chemical stimulus involved in sensory perception of pain [GO:0050968]